{
  "term_id": "GO:0005227",
  "gene": "UniProtKB:Q5T3F8",
  "term_label": "calcium-activated cation channel activity",
  "gene_name": "CSC1-like protein 2",
  "gene_symbol": "TMEM63B"
}